{
  "gene_name": "ELMO domain-containing protein 3",
  "gene_symbol": "ELMOD3",
  "gene": "UniProtKB:Q96FG2",
  "term_id": "GO:0005794",
  "term_label": "Golgi apparatus"
}